{
  "term_id": "GO:0005667",
  "gene_symbol": "HIF1A",
  "gene_name": "Hypoxia-inducible factor 1-alpha",
  "gene": "UniProtKB:Q16665",
  "term_label": "transcription regulator complex"
}